procentriole [GO:0120098] (cellular component) References: PMID:18620859, PMID:21289083, PMID:25047614 Sources: GOC:bhm, GOC:krc Definition: A cellular structure that is the site of a developing centriole, which will become a microtubule organizing center. During the canonical pathway of centriole duplication that occurs during the cell division cycle, procentrioles grow at the proximal ends of both mother and daughter centrioles. In the newly divided cells, the original mother and daughter centrioles become mother centrioles while the procentrioles become the new daughter centrioles. Procentrioles can also arise from de novo pathways that occur in multiciliated cells. In ciliated epithelial cells, numerous procentrioles arise form electron dense material referred to as fibrous granules and deuterosomes. The pathway of procentriole formation in multiciliated protists appears to be similar to that in mammalian multiciliated epithelium. In sperm of primitive land plants, multiple procentrioles are formed from a blepharoplast giving rise to multicilated sperm cells. Relationships: is a type of cellular anatomical structure [GO:0110165]; is part of cytoplasm [GO:0005737]